{
  "term_id": "GO:0000244",
  "gene": "UniProtKB:Q6P2Q9",
  "gene_symbol": "PRPF8",
  "gene_name": "Pre-mRNA-processing-splicing factor 8",
  "term_label": "spliceosomal tri-snRNP complex assembly"
}